positive regulation of muscle cell apoptotic process [GO:0010661] (biological process) Definition: Any process that increases the rate or frequency of muscle cell apoptotic process, a form of programmed cell death induced by external or internal signals that trigger the activity of proteolytic caspases whose actions dismantle a muscle cell and result in its death. Relationships: is a type of regulation of muscle cell apoptotic process [GO:0010660]; is a type of positive regulation of apoptotic process [GO:0043065]; positively regulates muscle cell apoptotic process [GO:0010657] Sources: GOC:dph, GOC:mtg_apoptosis, GOC:tb Subtypes: GO:0010663, positive regulation of smooth muscle cell apoptotic process [GO:0034393] Also known as: positive regulation of muscle cell apoptosis